{
  "gene_symbol": "RIBC2",
  "gene": "UniProtKB:Q9H4K1",
  "term_id": "UNKNOWN:0001",
  "gene_name": "RIB43A-like with coiled-coils protein 2",
  "term_label": "Unknown molecular function"
}